{
  "gene_name": "Epidermal growth factor receptor kinase substrate 8-like protein 3",
  "term_label": "ruffle membrane",
  "term_id": "GO:0032587",
  "gene": "UniProtKB:Q8TE67",
  "gene_symbol": "EPS8L3"
}